L-threonine catabolic process [GO:0006567] (biological process) Subtypes: L-threonine catabolic process to D-lactate [GO:0019517], L-threonine catabolic process to glycine [GO:0019518], L-threonine catabolic process to propionate [GO:0070689], L-threonine catabolic process to acetyl-CoA [GO:0070690] Relationships: is a type of threonine metabolic process [GO:0006566]; is a type of L-amino acid catabolic process [GO:0170035]; is a type of proteinogenic amino acid catabolic process [GO:0170040] Sources: GOC:jl, ISBN:0198506732 Also known as: threonine breakdown, threonine catabolism, threonine degradation Definition: The chemical reactions and pathways resulting in the breakdown of L-threonine (2-amino-3-hydroxybutyric acid), a polar, uncharged, essential amino acid found in peptide linkage in proteins.